{
  "term_label": "Unknown biological process",
  "gene_symbol": "A0A499FJF3",
  "gene_name": "Rho-GAP domain-containing protein",
  "gene": "UniProtKB:A0A499FJF3",
  "term_id": "UNKNOWN:0002"
}